3-cyano-L-alanine catabolic process [GO:1903559] (biological process) References: PMID:24100226, PMID:24843024 Sources: GOC:TermGenie, GOC:kmv, GO_REF:0000068 Relationships: is a type of GO:0050899; is a type of L-amino acid catabolic process [GO:0170035]; is a type of non-proteinogenic amino acid catabolic process [GO:0170044] Also known as: 3-cyano-L-alanine breakdown, 3-cyano-L-alanine catabolism, 3-cyano-L-alanine degradation Definition: The chemical reactions and pathways resulting in the breakdown of 3-cyano-L-alanine.